{
  "term_label": "mitochondrial membrane",
  "gene": "UniProtKB:Q9NYZ2",
  "term_id": "GO:0031966",
  "gene_symbol": "SLC25A37",
  "gene_name": "Mitoferrin-1"
}